{
  "gene": "UniProtKB:Q6ZNC8",
  "term_label": "acyltransferase activity",
  "gene_name": "Lysophospholipid acyltransferase 1",
  "gene_symbol": "MBOAT1",
  "term_id": "GO:0016746"
}